{
  "gene_name": "Homocysteine-responsive endoplasmic reticulum-resident ubiquitin-like domain member 2 protein",
  "term_label": "endoplasmic reticulum unfolded protein response",
  "gene": "UniProtKB:Q9BSE4",
  "term_id": "GO:0030968",
  "gene_symbol": "HERPUD2"
}